{
  "gene_symbol": "IFITM2",
  "term_label": "host-mediated suppression of symbiont invasion",
  "gene": "UniProtKB:Q01629",
  "gene_name": "Interferon-induced transmembrane protein 2",
  "term_id": "GO:0046597"
}